{
  "gene_name": "Endogenous retrovirus group K member 24 Gag polyprotein",
  "gene": "UniProtKB:P63145",
  "term_label": "Unknown molecular function",
  "term_id": "UNKNOWN:0001",
  "gene_symbol": "ERVK-24"
}